{
  "term_label": "nucleoside diphosphate kinase activity",
  "term_id": "GO:0004550",
  "gene": "UniProtKB:P23919",
  "gene_name": "Thymidylate kinase",
  "gene_symbol": "DTYMK"
}